{
  "term_id": "GO:0004984",
  "term_label": "olfactory receptor activity",
  "gene_symbol": "OR6X1",
  "gene_name": "Olfactory receptor 6X1",
  "gene": "UniProtKB:Q8NH79"
}